{
  "term_id": "UNKNOWN:0001",
  "gene_symbol": "C2CD4D",
  "gene": "UniProtKB:B7Z1M9",
  "gene_name": "C2 calcium-dependent domain-containing protein 4D",
  "term_label": "Unknown molecular function"
}